{
  "term_label": "positive regulation of apoptotic process",
  "gene_symbol": "TGM2",
  "gene": "UniProtKB:P21980",
  "gene_name": "Protein-glutamine gamma-glutamyltransferase 2",
  "term_id": "GO:0043065"
}